{
  "gene_symbol": "PCSK7",
  "term_label": "Golgi membrane",
  "gene": "UniProtKB:Q16549",
  "gene_name": "Proprotein convertase subtilisin_kexin type 7",
  "term_id": "GO:0000139"
}